 [IAO:0000116]